{
  "term_label": "DNA cytosine deamination",
  "gene": "UniProtKB:Q96AK3",
  "term_id": "GO:0070383",
  "gene_symbol": "APOBEC3D",
  "gene_name": "DNA dC-dU-editing enzyme APOBEC-3D"
}